{
  "gene_symbol": "AMY2B",
  "term_label": "extracellular space",
  "gene_name": "Alpha-amylase 2B",
  "gene": "UniProtKB:P19961",
  "term_id": "GO:0005615"
}